{
  "gene": "UniProtKB:P28067",
  "term_id": "GO:0019886",
  "term_label": "antigen processing and presentation of exogenous peptide antigen via MHC class II",
  "gene_symbol": "HLA-DMA",
  "gene_name": "HLA class II histocompatibility antigen, DM alpha chain"
}